{
  "gene_symbol": "PRPF8",
  "gene": "UniProtKB:Q6P2Q9",
  "term_id": "GO:0030620",
  "gene_name": "Pre-mRNA-processing-splicing factor 8",
  "term_label": "U2 snRNA binding"
}